ribulose bisphosphate carboxylase complex [GO:0048492] (cellular component) Definition: A complex containing either both large and small subunits or just small subunits which carries out the activity of producing 3-phosphoglycerate from carbon dioxide and ribulose-1,5-bisphosphate. Sources: GOC:mlg Also known as: RubisCO complex Subtypes: chloroplast ribulose bisphosphate carboxylase complex [GO:0009573], chromatophore ribulose bisphosphate carboxylase complex [GO:0048494] Relationships: is a type of catalytic complex [GO:1902494]; is part of GO:0005737